3-methylbut-2-enoyl-CoA(4-) biosynthetic process [GO:1902200] (biological process) References: PMID:11231285 Sources: GOC:TermGenie Also known as: 3-methylbut-2-enoyl-CoA(4-) anabolism, 3-methylbut-2-enoyl-CoA(4-) biosynthesis, 3-methylbut-2-enoyl-CoA(4-) formation, 3-methylbut-2-enoyl-CoA(4-) synthesis Relationships: is a type of fatty-acyl-CoA biosynthetic process [GO:0046949]; is a type of 3-methylbut-2-enoyl-CoA(4-) metabolic process [GO:1902198] Definition: The chemical reactions and pathways resulting in the formation of 3-methylbut-2-enoyl-CoA(4-).